{
  "term_id": "GO:0042908",
  "gene": "UniProtKB:P33527",
  "gene_name": "Multidrug resistance-associated protein 1",
  "term_label": "xenobiotic transport",
  "gene_symbol": "ABCC1"
}